{
  "term_id": "GO:0051028",
  "gene_symbol": "HNRNPA2B1",
  "gene_name": "Heterogeneous nuclear ribonucleoproteins A2_B1",
  "term_label": "mRNA transport",
  "gene": "UniProtKB:P22626"
}